{
  "gene_symbol": "HSP90AA2P",
  "gene": "UniProtKB:Q14568",
  "gene_name": "Heat shock protein HSP 90-alpha A2",
  "term_label": "ATP binding",
  "term_id": "GO:0005524"
}